{
  "gene": "UniProtKB:P98177",
  "term_id": "GO:0000981",
  "gene_symbol": "FOXO4",
  "term_label": "DNA-binding transcription factor activity, RNA polymerase II-specific",
  "gene_name": "Forkhead box protein O4"
}